{
  "gene_name": "Sodium channel subunit beta-4",
  "term_label": "voltage-gated sodium channel complex",
  "gene_symbol": "SCN4B",
  "gene": "UniProtKB:Q8IWT1",
  "term_id": "GO:0001518"
}